{
  "term_id": "GO:1990837",
  "gene_symbol": "SHOX",
  "gene": "UniProtKB:O15266",
  "gene_name": "Short stature homeobox protein",
  "term_label": "sequence-specific double-stranded DNA binding"
}